{
  "gene_name": "Uncharacterized protein C8orf48",
  "term_label": "Unknown molecular function",
  "term_id": "UNKNOWN:0001",
  "gene": "UniProtKB:Q96LL4",
  "gene_symbol": "C8orf48"
}